regulation of Notch signaling pathway [GO:0008593] (biological process) Also known as: regulation of N signaling pathway, regulation of N signalling pathway, regulation of Notch signalling pathway Definition: Any process that modulates the frequency, rate or extent of the Notch signaling pathway. Subtypes: negative regulation of Notch signaling pathway [GO:0045746], GO:0045747, regulation of Notch signaling pathway involved in somitogenesis [GO:1902366] Sources: GOC:go_curators Relationships: is a type of GO:0009966; RO_0002211 Notch signaling pathway [GO:0007219]